{
  "term_id": "GO:0005737",
  "gene_name": "Cold shock domain-containing protein C2",
  "gene": "UniProtKB:Q9Y534",
  "gene_symbol": "CSDC2",
  "term_label": "cytoplasm"
}